{
  "gene_name": "Putative ATP-dependent RNA helicase DDX11-like protein 8",
  "gene_symbol": "DDX11L8",
  "gene": "UniProtKB:A8MPP1",
  "term_id": "GO:0034085",
  "term_label": "establishment of sister chromatid cohesion"
}